{
  "gene_symbol": "RBMXL1",
  "term_label": "mRNA splicing, via spliceosome",
  "gene_name": "RNA binding motif protein, X-linked-like-1",
  "gene": "UniProtKB:Q96E39",
  "term_id": "GO:0000398"
}